netrin receptor binding [GO:1990890] (molecular function) Relationships: is a type of signaling receptor binding [GO:0005102]; is part of netrin-activated signaling pathway [GO:0038007] References: PMID:8861902, PMID:9126742 Sources: GOC:kmv Definition: Binding to a netrin receptor.